{
  "gene": "UniProtKB:Q8NCU1",
  "gene_symbol": "CCDC197",
  "term_label": "Unknown biological process",
  "gene_name": "Uncharacterized protein CCDC197",
  "term_id": "UNKNOWN:0002"
}